{
  "gene_symbol": "OR5W2",
  "term_id": "UNKNOWN:0002",
  "term_label": "Unknown biological process",
  "gene": "UniProtKB:Q8NH69",
  "gene_name": "Olfactory receptor 5W2"
}